{
  "gene_name": "Integrin beta-6",
  "term_label": "cell surface",
  "gene_symbol": "ITGB6",
  "gene": "UniProtKB:P18564",
  "term_id": "GO:0009986"
}